{
  "term_id": "UNKNOWN:0002",
  "gene_symbol": "SLC66A3",
  "gene": "UniProtKB:Q8N755",
  "term_label": "Unknown biological process",
  "gene_name": "Solute carrier family 66 member 3"
}